sexual spore wall [GO:0097514] (cellular component) Definition: A specialized envelope lying outside the cell membrane of a spore derived from a product of meiosis. Sources: GOC:cjm, GOC:mah Relationships: is a type of spore wall [GO:0031160]